host cell Cajal body [GO:0072495] (cellular component) Relationships: is a type of host cell nuclear part [GO:0044094]; is part of GO:0044095 Definition: A class of nuclear body in the eukaryotic host cell, first seen after silver staining by Ramon y Cajal in 1903, enriched in small nuclear ribonucleoproteins, and certain general RNA polymerase II transcription factors; ultrastructurally, they appear as a tangle of coiled, electron-dense threads roughly 0.5 micrometers in diameter; involved in aspects of snRNP biogenesis; the protein coilin serves as a marker for Cajal bodies. Some argue that Cajal bodies are the sites for preassembly of transcriptosomes, unitary particles involved in transcription and processing of RNA. The host is the larger of the organisms involved in a symbiotic interaction. Sources: GOC:rph Also known as: coiled body of host, host cell coiled body